interleukin-18 receptor binding [GO:0045515] (molecular function) Also known as: IL-18, interleukin-18 receptor ligand Definition: Binding to an interleukin-18 receptor. Relationships: is a type of cytokine receptor binding [GO:0005126] Sources: GOC:go_curators